{
  "gene_symbol": "DUSP9",
  "gene_name": "Dual specificity protein phosphatase 9",
  "gene": "UniProtKB:Q99956",
  "term_label": "cytosol",
  "term_id": "GO:0005829"
}